{
  "gene_name": "Large ribosomal subunit protein uL2m",
  "gene_symbol": "MRPL2",
  "gene": "UniProtKB:Q5T653",
  "term_label": "mitochondrial large ribosomal subunit",
  "term_id": "GO:0005762"
}